{
  "gene_symbol": "EIF4EBP1",
  "gene": "UniProtKB:Q13541",
  "term_label": "translation repressor activity",
  "term_id": "GO:0030371",
  "gene_name": "Eukaryotic translation initiation factor 4E-binding protein 1"
}